{
  "gene": "UniProtKB:O95613",
  "term_label": "mitotic spindle organization",
  "gene_name": "Pericentrin",
  "term_id": "GO:0007052",
  "gene_symbol": "PCNT"
}